regulation of cytoplasmic translational initiation [GO:1904688] (biological process) Subtypes: GO:1901193, regulation of cap-dependent translational initiation [GO:1903674], regulation of cap-independent translational initiation [GO:1903677], negative regulation of cytoplasmic translational initiation [GO:1904689], positive regulation of cytoplasmic translational initiation [GO:1904690], regulation of cytoplasmic translational initiation in response to stress [GO:1990611] Relationships: is a type of regulation of translational initiation [GO:0006446]; is a type of regulation of cytoplasmic translation [GO:2000765]; regulates cytoplasmic translational initiation [GO:0002183] Definition: Any process that modulates the frequency, rate or extent of cytoplasmic translational initiation. References: PMID:12242291 Sources: GOC:TermGenie, GO_REF:0000058